{
  "term_id": "GO:0006874",
  "term_label": "intracellular calcium ion homeostasis",
  "gene_name": "Sarcoplasmic_endoplasmic reticulum calcium ATPase 2",
  "gene": "UniProtKB:P16615",
  "gene_symbol": "ATP2A2"
}